{
  "gene_name": "Phosphatidylinositol 4-phosphate 3-kinase C2 domain-containing subunit alpha",
  "term_id": "GO:0035005",
  "term_label": "1-phosphatidylinositol-4-phosphate 3-kinase activity",
  "gene": "UniProtKB:O00443",
  "gene_symbol": "PIK3C2A"
}